{
  "gene_symbol": "TMEM54",
  "term_label": "Unknown molecular function",
  "gene": "UniProtKB:Q969K7",
  "term_id": "UNKNOWN:0001",
  "gene_name": "Transmembrane protein 54"
}